NLS-bearing protein import into nucleus [GO:0006607] (biological process) Sources: GOC:ai Definition: The directed movement of a protein bearing a nuclear localization signal (NLS) from the cytoplasm into the nucleus, across the nuclear envelope. Also known as: NLS-bearing substrate import into cell nucleus, NLS-bearing substrate import into nucleus, NLS-bearing substrate transport from cytoplasm to nucleus, NLS-bearing substrate-nucleus import Relationships: is a type of protein import into nucleus [GO:0006606]